dorsal spinal cord interneuron posterior axon guidance [GO:0097379] (biological process) Relationships: is a type of GO:0033564; is a type of GO:0097378 References: PMID:19545367 Sources: GOC:yaf Definition: The process in which the migration of an axon growth cone of a dorsal spinal cord interneuron is directed to a specific target site in the posterior direction along the anterior-posterior body axis in response to a combination of attractive and repulsive cues. The anterior-posterior axis is defined by a line that runs from the head or mouth of an organism to the tail or opposite end of the organism. Also known as: dorsal interneuron caudal axon projection